{
  "gene_name": "Hepatocyte nuclear factor 3-gamma",
  "term_id": "GO:0009653",
  "gene": "UniProtKB:P55318",
  "gene_symbol": "FOXA3",
  "term_label": "anatomical structure morphogenesis"
}